interphase microtubule organizing center assembly [GO:0031024] (biological process) References: PMID:15068790 Sources: GOC:mah Also known as: interphase microtubule organising center biosynthesis, interphase microtubule organising center formation, interphase microtubule organizing centre assembly, interphase microtubule organizing center biogenesis Relationships: is a type of GO:0022607; is a type of microtubule organizing center organization [GO:0031023] Definition: The aggregation, arrangement and bonding together of a set of components, including gamma-tubulin and other proteins, to form an interphase microtubule organizing center.